{
  "gene_name": "Ras-related C3 botulinum toxin substrate 1",
  "term_id": "GO:0060326",
  "term_label": "cell chemotaxis",
  "gene_symbol": "RAC1",
  "gene": "UniProtKB:P63000"
}